{
  "term_label": "dolichol-linked oligosaccharide biosynthetic process",
  "gene_symbol": "ALG8",
  "term_id": "GO:0006488",
  "gene_name": "Probable dolichyl pyrophosphate Glc1Man9GlcNAc2 alpha-1,3-glucosyltransferase",
  "gene": "UniProtKB:Q9BVK2"
}